{
  "gene_name": "U6 snRNA-associated Sm-like protein LSm5",
  "gene": "UniProtKB:Q9Y4Y9",
  "gene_symbol": "LSM5",
  "term_id": "GO:0003723",
  "term_label": "RNA binding"
}